lipid antigen binding [GO:0030882] (molecular function) Subtypes: endogenous lipid antigen binding [GO:0030883], exogenous lipid antigen binding [GO:0030884] References: PMID:14500461 Definition: Binding to a lipid antigen. Relationships: is_a GO:0003823; is a type of GO:0008289